{
  "gene": "UniProtKB:A0A5F9ZHU2",
  "gene_symbol": "A0A5F9ZHU2",
  "term_label": "Unknown biological process",
  "gene_name": "Uncharacterized protein",
  "term_id": "UNKNOWN:0002"
}